{
  "gene": "UniProtKB:Q9BZD2",
  "term_id": "GO:0005886",
  "gene_name": "Equilibrative nucleoside transporter 3",
  "term_label": "plasma membrane",
  "gene_symbol": "SLC29A3"
}